renal urate salt excretion [GO:0097744] (biological process) Relationships: is_a renal tubular secretion [GO:0097254] Also known as: urate excretion, urate salt excretion Definition: The elimination of urate salt or uric acid from peritubular capillaries (or surrounding hemolymph in invertebrates) into the renal tubules to be incorporated subsequently into the urine. References: PMID:25287933, PMID:3906799 Sources: GOC:jl, Wikipedia:Renal_physiology#Secretion